regulation of membrane repolarization during atrial cardiac muscle cell action potential [GO:1905000] (biological process) Subtypes: negative regulation of membrane repolarization during atrial cardiac muscle cell action potential [GO:1905001], positive regulation of membrane repolarization during atrial cardiac muscle cell action potential [GO:1905002] Relationships: is a type of GO:0060372; is a type of regulation of membrane repolarization during cardiac muscle cell action potential [GO:1905031]; regulates membrane repolarization during atrial cardiac muscle cell action potential [GO:0098914] Definition: Any process that modulates the frequency, rate or extent of membrane repolarization during atrial cardiac muscle cell action potential. Also known as: regulation of atrial repolarization, regulation of electrocardiogram QRS complex References: PMID:21098446 Sources: GOC:BHF, GOC:BHF_miRNA, GOC:TermGenie, GOC:mtg_cardiac_conduct_nov11, GOC:rph